{
  "term_id": "GO:0050870",
  "term_label": "positive regulation of T cell activation",
  "gene_name": "Tyrosine-protein phosphatase non-receptor type substrate 1",
  "gene": "UniProtKB:P78324",
  "gene_symbol": "SIRPA"
}